UDP-alpha-D-glucose biosynthetic process [GO:0120530] (biological process) Sources: MetaCyc:PWY-7343 Also known as: UDP-D-glucose biosynthesis, UDP-D-glucose biosynthetic process, UDP-glucose biosynthesis, uridine diphosphate glucose biosynthesis, uridine diphosphate glucose biosynthetic process Relationships: is a type of UDP-alpha-D-glucose metabolic process [GO:0006011]; is a type of nucleotide-sugar biosynthetic process [GO:0009226] Definition: The chemical reactions and pathways resulting in the formation of UDP-alpha-D-glucose, a substance composed of alpha-D-glucose in glycosidic linkage with uridine diphosphate.